somatic diversification of immunoglobulins [GO:0016445] (biological process) Relationships: is a type of somatic diversification of immune receptors [GO:0002200]; BFO_0000050 immunoglobulin production [GO:0002377] Subtypes: gene conversion of immunoglobulin genes [GO:0002206], GO:0002208, alternate splicing of immunoglobulin genes [GO:0002564], somatic diversification of immunoglobulin genes by N region addition [GO:0002570], somatic hypermutation of immunoglobulin genes [GO:0016446], somatic recombination of immunoglobulin gene segments [GO:0016447] Sources: GOC:add, GOC:ma, ISBN:0781735149 Definition: The somatic process that results in the generation of sequence diversity of immunoglobulins. Also known as: somatic diversification of antibodies